{
  "term_id": "UNKNOWN:0001",
  "gene_name": "Mitogen-activated protein kinase kinase kinase 4",
  "gene_symbol": "MAP3K4",
  "gene": "UniProtKB:Q9Y6R4",
  "term_label": "Unknown molecular function"
}